{
  "term_id": "GO:0000795",
  "term_label": "synaptonemal complex",
  "gene": "UniProtKB:Q8IZU1",
  "gene_name": "Protein FAM9A",
  "gene_symbol": "FAM9A"
}